{
  "gene": "UniProtKB:O00629",
  "term_label": "nucleus",
  "gene_name": "Importin subunit alpha-3",
  "term_id": "GO:0005634",
  "gene_symbol": "KPNA4"
}